{
  "gene_symbol": "AMER2",
  "term_label": "plasma membrane",
  "term_id": "GO:0005886",
  "gene_name": "APC membrane recruitment protein 2",
  "gene": "UniProtKB:Q8N7J2"
}